{
  "gene_symbol": "PCDHGA11",
  "term_label": "cell adhesion molecule binding",
  "term_id": "GO:0050839",
  "gene_name": "Protocadherin gamma-A11",
  "gene": "UniProtKB:Q9Y5H2"
}